{
  "gene": "UniProtKB:Q13115",
  "gene_name": "Dual specificity protein phosphatase 4",
  "term_label": "phosphoprotein phosphatase activity",
  "gene_symbol": "DUSP4",
  "term_id": "GO:0004721"
}